MCM complex assembly [GO:0072689] (biological process) References: PMID:21813639 Sources: GOC:mah Definition: The aggregation, arrangement and bonding together of a set of components to form an MCM complex, a hexameric protein complex required for the initiation and regulation of DNA replication. Relationships: is a type of protein-containing complex assembly [GO:0065003]